{
  "gene": "UniProtKB:O43617",
  "gene_name": "Trafficking protein particle complex subunit 3",
  "gene_symbol": "TRAPPC3",
  "term_label": "guanyl-nucleotide exchange factor activity",
  "term_id": "GO:0005085"
}